{
  "gene_symbol": "ETAA1",
  "gene_name": "Ewing's tumor-associated antigen 1",
  "term_id": "GO:2000001",
  "gene": "UniProtKB:Q9NY74",
  "term_label": "regulation of DNA damage checkpoint"
}